{
  "gene": "UniProtKB:Q9NQW1",
  "gene_symbol": "SEC31B",
  "term_label": "COPII vesicle coat",
  "term_id": "GO:0030127",
  "gene_name": "Protein transport protein Sec31B"
}